{
  "gene_name": "Neuronal acetylcholine receptor subunit alpha-10",
  "term_id": "GO:0043005",
  "term_label": "neuron projection",
  "gene_symbol": "CHRNA10",
  "gene": "UniProtKB:Q9GZZ6"
}